{
  "gene_symbol": "PHC1",
  "gene_name": "Polyhomeotic-like protein 1",
  "term_label": "nucleus",
  "gene": "UniProtKB:P78364",
  "term_id": "GO:0005634"
}